centrosome-templated microtubule nucleation [GO:0090222] (biological process) Sources: GOC:ascb_2009, GOC:dph, GOC:tb Definition: The 'de novo' formation of a microtubule, in which tubulin heterodimers form metastable oligomeric aggregates from the centrosome. Relationships: is a type of microtubule nucleation by microtubule organizing center [GO:0051418]